{
  "gene_name": "HAUS augmin-like complex subunit 2",
  "term_id": "GO:0051225",
  "gene": "UniProtKB:Q9NVX0",
  "gene_symbol": "HAUS2",
  "term_label": "spindle assembly"
}